{
  "term_id": "GO:0003073",
  "gene": "UniProtKB:P07288",
  "gene_name": "Prostate-specific antigen",
  "term_label": "regulation of systemic arterial blood pressure",
  "gene_symbol": "KLK3"
}